diadenosine tetraphosphate catabolic process [GO:0015967] (biological process) Definition: The chemical reactions and pathways resulting in the breakdown of diadenosine tetraphosphate, a derivative of the nucleoside adenosine with four phosphate groups attached. Relationships: is a type of diadenosine polyphosphate catabolic process [GO:0015961] Also known as: diadenosine tetraphosphate breakdown, diadenosine tetraphosphate catabolism, diadenosine tetraphosphate degradation Sources: GOC:ai